{
  "term_id": "GO:0007080",
  "gene_name": "Histone H3.Y",
  "term_label": "mitotic metaphase chromosome alignment",
  "gene_symbol": "H3Y1",
  "gene": "UniProtKB:P0DPK2"
}